{
  "gene_symbol": "SLC4A8",
  "gene_name": "Electroneutral sodium bicarbonate exchanger 1",
  "gene": "UniProtKB:Q2Y0W8",
  "term_id": "GO:0055085",
  "term_label": "transmembrane transport"
}